{
  "gene": "UniProtKB:Q8NGS0",
  "term_id": "GO:0007165",
  "gene_symbol": "OR1N1",
  "term_label": "signal transduction",
  "gene_name": "Olfactory receptor 1N1"
}